ESCRT-0 complex [GO:0033565] (cellular component) References: PMID:12055639, PMID:17543868 Sources: GOC:rb Definition: A protein complex required for the recycling of Golgi proteins, formation of lumenal membranes and sorting of ubiquitinated proteins into those membranes. This complex includes Vps1p and Hse1p in yeast and the Hrs and STAM proteins in mammals. Relationships: is a type of ESCRT complex [GO:0036452] Also known as: Hrs/STAM complex, Vps27p-Hse1p complex